{
  "term_label": "DNA-binding transcription factor activity, RNA polymerase II-specific",
  "gene_name": "SKI family transcriptional corepressor 2",
  "gene": "UniProtKB:Q2VWA4",
  "gene_symbol": "SKOR2",
  "term_id": "GO:0000981"
}